{
  "gene": "UniProtKB:Q149N8",
  "gene_symbol": "SHPRH",
  "term_id": "UNKNOWN:0003",
  "term_label": "Unknown cellular component",
  "gene_name": "E3 ubiquitin-protein ligase SHPRH"
}